regulation of neutrophil extravasation [GO:2000389] (biological process) Definition: Any process that modulates the frequency, rate or extent of neutrophil extravasation. Relationships: is_a regulation of cellular extravasation [GO:0002691]; is a type of regulation of neutrophil migration [GO:1902622]; RO_0002211 GO:0072672 Subtypes: negative regulation of neutrophil extravasation [GO:2000390], positive regulation of neutrophil extravasation [GO:2000391] Sources: GOC:mah